{
  "gene_name": "Copper-transporting ATPase 1",
  "gene_symbol": "ATP7A",
  "term_label": "copper ion binding",
  "term_id": "GO:0005507",
  "gene": "UniProtKB:Q04656"
}